{
  "gene_symbol": "NRARP",
  "gene_name": "Notch-regulated ankyrin repeat-containing protein",
  "gene": "UniProtKB:Q7Z6K4",
  "term_label": "Unknown molecular function",
  "term_id": "UNKNOWN:0001"
}